{
  "gene_symbol": "FADS2",
  "term_label": "oxidoreductase activity, acting on paired donors, with oxidation of a pair of donors resulting in the reduction of molecular oxygen to two molecules of water",
  "term_id": "GO:0016717",
  "gene": "UniProtKB:O95864",
  "gene_name": "Acyl-CoA 6-desaturase"
}